cyanelle stroma [GO:0034060] (cellular component) Sources: GOC:rph Definition: The space enclosed by the double membrane of a cyanelle. Relationships: is a type of plastid stroma [GO:0009532]; is part of cyanelle [GO:0009842]